regulation of penicillin biosynthetic process [GO:1900196] (biological process) Sources: GOC:TermGenie, GOC:di Definition: Any process that modulates the frequency, rate or extent of penicillin biosynthetic process. Also known as: regulation of penicillin anabolism, regulation of penicillin biosynthesis, regulation of penicillin formation, regulation of penicillin synthesis Relationships: is a type of regulation of amide metabolic process [GO:0034248]; is a type of regulation of sulfur metabolic process [GO:0042762]; is a type of regulation of small molecule metabolic process [GO:0062012]; is a type of regulation of secondary metabolite biosynthetic process [GO:1900376]; regulates penicillin biosynthetic process [GO:0042318] Subtypes: negative regulation of penicillin biosynthetic process [GO:1900197], positive regulation of penicillin biosynthetic process [GO:1900198]